glucuronosyltransferase activity [GO:0015020] (molecular function) Also known as: 1-naphthol glucuronyltransferase activity, 1-naphthol-UDP-glucuronosyltransferase activity, 17-OH steroid UDPGT activity, 17-beta-hydroxysteroid UDP-glucuronosyltransferase activity, 17beta-hydroxysteroid UDP-glucuronosyltransferase activity, 3-OH androgenic UDPGT activity, 3-alpha-hydroxysteroid UDP-glucuronosyltransferase activity, 3alpha-hydroxysteroid UDP-glucuronosyltransferase activity, 4-hydroxybiphenyl UDP-glucuronosyltransferase activity, 4-methylumbelliferone UDP-glucuronosyltransferase activity, 4-nitrophenol UDP-glucuronyltransferase activity, 4-nitrophenol UDPGT activity, UDP glucuronate-estradiol-glucuronosyltransferase activity, UDP glucuronate-estriol glucuronosyltransferase activity, UDP-glucuronate-4-hydroxybiphenyl glucuronosyltransferase activity, UDP-glucuronate-bilirubin glucuronyltransferase activity, UDPglucuronate beta-D-glucuronosyltransferase (acceptor-unspecific) activity, bilirubin UDP-glucuronosyltransferase activity, bilirubin UDPGT activity, bilirubin glucuronyltransferase activity, bilirubin monoglucuronide glucuronyltransferase activity, bilirubin uridine diphosphoglucuronyltransferase activity, ciramadol UDP-glucuronyltransferase activity, estriol UDPglucuronosyltransferase activity, estrone UDPglucuronosyltransferase activity, morphine glucuronyltransferase activity, p-hydroxybiphenyl UDP glucuronyltransferase activity, p-nitrophenol UDP-glucuronosyltransferase activity, p-nitrophenol UDP-glucuronyltransferase activity, p-nitrophenylglucuronosyltransferase activity, p-phenylphenol glucuronyltransferase activity, phenyl-UDP-glucuronosyltransferase activity, pnp-UDPGT activity, uridine diphosphoglucuronate-1,2-diacylglycerol glucuronosyltransferase activity, uridine diphosphoglucuronate-4-hydroxybiphenyl glucuronosyltransferase activity, uridine diphosphoglucuronate-bilirubin glucuronoside glucuronosyltransferase activity, uridine diphosphoglucuronate-bilirubin glucuronosyltransferase activity, uridine diphosphoglucuronate-estradiol glucuronosyltransferase activity, uridine diphosphoglucuronate-estriol 16-alpha-glucuronosyltransferase activity, uridine diphosphoglucuronate-estriol 16alpha-glucuronosyltransferase activity, uridine diphosphoglucuronate-estriol glucuronosyltransferase activity, GT activity, PNP-UDPGT, UDP glucuronic acid transferase activity, UDP glucuronosyltransferase activity, UDP glucuronyltransferase activity, UDP-glucuronate beta-D-glucuronosyltransferase (acceptor-unspecific), UDP-glucuronosyltransferase activity, UDP-glucuronyltransferase activity, UDPGA transferase activity, UDPGA-glucuronyltransferase activity, UDPGT activity, uridine 5'-diphosphoglucuronyltransferase activity, uridine diphosphate glucuronyltransferase activity, uridine diphosphoglucuronosyltransferase activity, uridine diphosphoglucuronyltransferase activity Definition: Catalysis of the reaction: glucuronate acceptor + UDP-alpha-D-glucuronate = acceptor beta-D-glucuronoside + H+ + UDP. Subtypes: galactosylgalactosylxylosylprotein 3-beta-glucuronosyltransferase activity [GO:0015018], N-acetyllactosamine beta-1,3-glucuronosyltransferase activity [GO:0046987], asioloorosomucoid beta-1,3-glucuronosyltransferase activity [GO:0046988], galactosyl beta-1,3 N-acetylgalactosamine beta-1,3-glucuronosyltransferase activity [GO:0046989], luteolin-7-O-glucuronide 7-O-glucuronosyltransferase activity [GO:0047246], GO:0047247, bilirubin-glucuronoside glucuronosyltransferase activity [GO:0047278], luteolin 7-O-glucuronosyltransferase activity [GO:0050064], N-acetylglucosaminyl-proteoglycan 4-beta-glucuronosyltransferase activity [GO:0050509], N-acetylgalactosaminyl-proteoglycan 3-beta-glucuronosyltransferase activity [GO:0050510], glucuronoxylan glucuronosyltransferase activity [GO:0080116] Sources: RHEA:21032 Relationships: is a type of UDP-glycosyltransferase activity [GO:0008194]; is a type of hexosyltransferase activity [GO:0016758]